{
  "term_id": "GO:1905606",
  "gene": "UniProtKB:Q6PJG9",
  "gene_name": "Leucine-rich repeat and fibronectin type-III domain-containing protein 4",
  "gene_symbol": "LRFN4",
  "term_label": "regulation of presynapse assembly"
}